methane biosynthetic process from methanol and hydrogen [GO:1990491] (biological process) Also known as: methane biosynthesis from methanol and hydrogen, methanogenesis from methanol and hydrogen References: PMID:16347126 Sources: GOC:mengo_curators Definition: The chemical reactions and pathways resulting in the formation of methane from methanol and hydrogen. Relationships: is a type of methanogenesis, from methanol [GO:0019387]; is a type of hydrogen metabolic process [GO:1902421]